{
  "term_id": "GO:0003714",
  "term_label": "transcription corepressor activity",
  "gene_symbol": "IRF2BP2",
  "gene_name": "Interferon regulatory factor 2-binding protein 2",
  "gene": "UniProtKB:Q7Z5L9"
}